{
  "term_label": "regulation of transcription by RNA polymerase II",
  "gene_symbol": "PHF20",
  "term_id": "GO:0006357",
  "gene_name": "PHD finger protein 20",
  "gene": "UniProtKB:Q9BVI0"
}